{
  "term_id": "GO:0006355",
  "gene": "UniProtKB:O14744",
  "term_label": "regulation of DNA-templated transcription",
  "gene_symbol": "PRMT5",
  "gene_name": "Protein arginine N-methyltransferase 5"
}